co-transcriptional mRNA 3'-end processing, cleavage and polyadenylation pathway [GO:0180010] (biological process) References: PMID:31499460 Relationships: is a type of mRNA 3'-end processing [GO:0031124]; is a type of co-transcriptional RNA 3'-end processing, cleavage and polyadenylation pathway [GO:0180012] Definition: Any process involved in transcription termination-coupled 3' processing of RNA polymerase II mRNA transcripts by the 3' end cleavage and addition of a poly(A) tail. Also known as: cotranscriptional 3' processing of RNA polymerase II mRNA transcripts, mRNA polyadenylation